{
  "term_label": "Unknown biological process",
  "term_id": "UNKNOWN:0002",
  "gene_name": "Probable E3 ubiquitin-protein ligase HECTD2",
  "gene_symbol": "HECTD2",
  "gene": "UniProtKB:Q5U5R9"
}